{
  "gene": "UniProtKB:Q5TDH0",
  "gene_symbol": "DDI2",
  "term_id": "GO:0010498",
  "term_label": "proteasomal protein catabolic process",
  "gene_name": "Protein DDI1 homolog 2"
}